{
  "gene_name": "T cell receptor beta joining 1-4",
  "term_id": "UNKNOWN:0002",
  "term_label": "Unknown biological process",
  "gene_symbol": "TRBJ1-4",
  "gene": "UniProtKB:A0A0J9YXG5"
}